{
  "gene_symbol": "BIRC3",
  "gene": "UniProtKB:Q13489",
  "term_id": "GO:0061630",
  "term_label": "ubiquitin protein ligase activity",
  "gene_name": "Baculoviral IAP repeat-containing protein 3"
}